{
  "gene_name": "DNA topoisomerase 2-binding protein 1",
  "gene_symbol": "TOPBP1",
  "term_label": "BRCA1-B complex",
  "term_id": "GO:0070532",
  "gene": "UniProtKB:Q92547"
}